{
  "term_id": "UNKNOWN:0001",
  "gene_symbol": "SLITRK1",
  "gene": "UniProtKB:Q96PX8",
  "term_label": "Unknown molecular function",
  "gene_name": "SLIT and NTRK-like protein 1"
}